dichotomous subdivision of an epithelial terminal unit [GO:0060600] (BP) Sources: GOC:dph Definition: The process in which an epithelial cord, rod or tube bifurcates at its end. Also known as: primary branching of an epithelium Subtypes: dichotomous subdivision of terminal units involved in lung branching [GO:0060448], dichotomous subdivision of prostate epithelial cord terminal unit [GO:0060524], GO:0060598, GO:0060666, dichotomous subdivision of terminal units involved in ureteric bud branching [GO:0060678] Relationships: is a type of GO:0002009; is part of morphogenesis of a branching epithelium [GO:0061138]